{
  "term_id": "GO:0005096",
  "term_label": "GTPase activator activity",
  "gene": "UniProtKB:Q8IZ81",
  "gene_name": "ELMO domain-containing protein 2",
  "gene_symbol": "ELMOD2"
}